{
  "gene_symbol": "AMELX",
  "gene_name": "Amelogenin, X isoform",
  "term_label": "extracellular matrix",
  "term_id": "GO:0031012",
  "gene": "UniProtKB:Q99217"
}